ethanolamine biosynthetic process [GO:0046335] (biological process) Also known as: ethanolamine anabolism, ethanolamine biosynthesis, ethanolamine formation, ethanolamine synthesis Sources: GOC:ai Relationships: is a type of ethanolamine metabolic process [GO:0006580]; is a type of primary alcohol biosynthetic process [GO:0034309]; is a type of biogenic amine biosynthetic process [GO:0042401]; is a type of primary amino compound biosynthetic process [GO:1901162] Definition: The chemical reactions and pathways resulting in the formation of ethanolamine (2-aminoethanol), an important water-soluble base of phospholipid (phosphatidylethanolamine).